{
  "term_id": "GO:0005737",
  "gene_name": "Guanine nucleotide-binding protein G(i) subunit alpha-3",
  "gene_symbol": "GNAI3",
  "gene": "UniProtKB:P08754",
  "term_label": "cytoplasm"
}